{
  "gene": "UniProtKB:Q01954",
  "gene_name": "Zinc finger protein basonuclin-1",
  "gene_symbol": "BNC1",
  "term_label": "regulation of transcription by RNA polymerase I",
  "term_id": "GO:0006356"
}